L-serine transmembrane import into vacuole [GO:0090516] (biological process) Definition: The directed movement of L-serine into the vacuole across the vacuolar membrane. Relationships: is a type of GO:0015825; is a type of neutral amino acid transmembrane import into vacuole [GO:0034491]; is a type of L-alpha-amino acid transmembrane transport [GO:1902475] Sources: GOC:al